{
  "term_id": "GO:2000300",
  "gene_name": "Synaptic vesicle glycoprotein 2B",
  "gene": "UniProtKB:Q7L1I2",
  "gene_symbol": "SV2B",
  "term_label": "regulation of synaptic vesicle exocytosis"
}